positive regulation of chemokine (C-C motif) ligand 5 production [GO:0071651] (biological process) Relationships: is a type of GO:0032722; is a type of GO:0071649; positively regulates chemokine (C-C motif) ligand 5 production [GO:0071609] Definition: Any process that activates or increases the frequency, rate, or extent of production of chemokine (C-C motif) ligand 5. Also known as: positive regulation of CCL5 production, positive regulation of RANTES production, positive regulation of Regulated upon Activation, Normal T-cell Expressed, and Secreted production Sources: GOC:mah